{
  "term_id": "GO:0017147",
  "term_label": "Wnt-protein binding",
  "gene_symbol": "SFRP4",
  "gene": "UniProtKB:Q6FHJ7",
  "gene_name": "Secreted frizzled-related protein 4"
}